{
  "term_id": "UNKNOWN:0003",
  "gene": "UniProtKB:Q6UXR8",
  "gene_symbol": "UNQ6493_PRO21345",
  "gene_name": "Putative uncharacterized protein UNQ6493_PRO21345",
  "term_label": "Unknown cellular component"
}